{
  "term_label": "regulation of DNA-templated transcription",
  "gene": "UniProtKB:Q9BY66",
  "gene_name": "Lysine-specific demethylase 5D",
  "term_id": "GO:0006355",
  "gene_symbol": "KDM5D"
}